{
  "gene_symbol": "KDELR1",
  "term_id": "GO:0005783",
  "term_label": "endoplasmic reticulum",
  "gene": "UniProtKB:P24390",
  "gene_name": "ER lumen protein-retaining receptor 1"
}